Mon1-Ccz1 complex [GO:0035658] (CC) Relationships: is_a guanyl-nucleotide exchange factor complex [GO:0032045]; BFO_0000050 late endosome [GO:0005770] Definition: A protein complex that functions as a guanine nucleotide exchange factor (GEF) and converts Rab-GDP to Rab-GTP. In S. cerevisiae, this complex consists of at least Mon1 and Ccz1, and serves as a GEF for the Rab Ypt7p. References: PMID:20797862 Sources: GOC:rb